pyrimidine-containing compound transmembrane transport [GO:0072531] (biological process) Sources: GOC:mah Note: Note that this term is not intended for use in annotating lateral movement within membranes. Definition: The process in which a pyrimidine-containing compound is transported across a membrane. A pyrimidine-containing compound is any compound that contains pyrimidine or a formal derivative thereof. Also known as: pyrimidine-containing compound membrane transport Relationships: is a type of transmembrane transport [GO:0055085]; is a type of nitrogen compound transport [GO:0071705] Subtypes: GO:0015862, thiamine transmembrane transport [GO:0071934], GO:1904082, pyrimidine nucleotide import into mitochondrion [GO:1990519]